{
  "gene_symbol": "ENTREP1",
  "term_label": "Unknown biological process",
  "gene_name": "Endosomal transmembrane epsin interactor 1",
  "term_id": "UNKNOWN:0002",
  "gene": "UniProtKB:Q15884"
}